{
  "gene_symbol": "SLC35C2",
  "gene": "UniProtKB:Q9NQQ7",
  "gene_name": "Solute carrier family 35 member C2",
  "term_id": "GO:0005794",
  "term_label": "Golgi apparatus"
}